dextranase activity [GO:0033904] (molecular function) Definition: Catalysis of the endohydrolysis of 1,6-alpha-D-glucosidic linkages in dextran. Also known as: dextranase DL 2 activity, 1,6-alpha-D-glucan 6-glucanohydrolase activity, DL 2, alpha-1,6-glucan-6-glucanohydrolase activity, alpha-D-1,6-glucan-6-glucanohydrolase activity, dextran hydrolase activity, endo-dextranase activity, endodextranase activity Relationships: is a type of hydrolase activity, hydrolyzing O-glycosyl compounds [GO:0004553] Sources: EC:3.2.1.11